proximal/distal pattern formation involved in nephron development [GO:0072047] (biological process) Also known as: proximal-distal pattern formation involved in nephron development, proximal/distal nephron patterning Subtypes: proximal/distal pattern formation involved in mesonephric nephron development [GO:0061226], proximal/distal pattern formation involved in pronephric nephron development [GO:0072196], GO:0072272 Relationships: is a type of proximal/distal pattern formation [GO:0009954]; is a type of GO:0061004; is part of GO:0072006 Sources: GOC:mtg_kidney_jan10 Definition: The regionalization process in which specific areas of cell differentiation are determined along a proximal/distal axis of a nephron. The proximal/distal axis is defined by a line that runs from the center of the kidney (proximal end) outward (distal end).